positive regulation of protein oxidation [GO:1904808] (biological process) Relationships: is a type of positive regulation of protein modification process [GO:0031401]; is a type of regulation of protein oxidation [GO:1904806]; positively regulates protein oxidation [GO:0018158] References: PMID:22719267 Sources: GOC:TermGenie, GO_REF:0000058 Definition: Any process that activates or increases the frequency, rate or extent of protein oxidation. Also known as: positive regulation of protein amino acid oxidation, up regulation of protein amino acid oxidation, up regulation of protein oxidation, up-regulation of protein amino acid oxidation, up-regulation of protein oxidation, upregulation of protein amino acid oxidation, upregulation of protein oxidation, activation of protein amino acid oxidation, activation of protein oxidation